{
  "term_id": "UNKNOWN:0001",
  "term_label": "Unknown molecular function",
  "gene_name": "Smith-Magenis syndrome chromosomal region candidate gene 5 protein",
  "gene": "UniProtKB:Q8TEV8",
  "gene_symbol": "SMCR5"
}